{
  "term_id": "GO:0005739",
  "gene_name": "rRNA methyltransferase 2, mitochondrial",
  "gene": "UniProtKB:Q9UI43",
  "term_label": "mitochondrion",
  "gene_symbol": "MRM2"
}